lactation [GO:0007595] (biological process) Sources: ISBN:0198506732 Also known as: milk secretion Definition: The regulated release of milk from the mammary glands and the period of time that a mother lactates to feed her young. Regulation: regulated by regulation of lactation [GO:1903487]; negatively regulated by negative regulation of lactation [GO:1903488]; positively regulated by GO:1903489 Relationships: is a type of body fluid secretion [GO:0007589]; BFO_0000050 mammary gland development [GO:0030879]; has part milk ejection reflex [GO:0060156]